{
  "term_id": "UNKNOWN:0002",
  "gene_symbol": "PYROXD1",
  "gene": "UniProtKB:Q8WU10",
  "term_label": "Unknown biological process",
  "gene_name": "Pyridine nucleotide-disulfide oxidoreductase domain-containing protein 1"
}